{
  "term_label": "tetrahydrofolate metabolic process",
  "gene": "UniProtKB:Q99707",
  "term_id": "GO:0046653",
  "gene_symbol": "MTR",
  "gene_name": "Methionine synthase"
}